{
  "gene_name": "Butyrophilin-like protein 2",
  "gene_symbol": "BTNL2",
  "term_label": "regulation of cytokine production",
  "term_id": "GO:0001817",
  "gene": "UniProtKB:Q9UIR0"
}